{
  "term_label": "SCF-dependent proteasomal ubiquitin-dependent protein catabolic process",
  "gene_name": "F-box_WD repeat-containing protein 1A",
  "term_id": "GO:0031146",
  "gene_symbol": "BTRC",
  "gene": "UniProtKB:Q9Y297"
}